{
  "term_label": "Unknown cellular component",
  "gene": "UniProtKB:A0A1W2PRP0",
  "term_id": "UNKNOWN:0003",
  "gene_name": "Forkhead box protein L3",
  "gene_symbol": "FOXL3"
}